positive regulation of toll-like receptor 3 signaling pathway [GO:0034141] (biological process) Definition: Any process that activates or increases the frequency, rate, or extent of toll-like receptor 3 signaling pathway. Also known as: positive regulation of TLR3 signaling pathway, positive regulation of toll-like receptor 3 signalling pathway Relationships: is a type of regulation of toll-like receptor 3 signaling pathway [GO:0034139]; is a type of GO:0062208; is a type of positive regulation of intracellular signal transduction [GO:1902533]; positively regulates GO:0034138 References: PMID:16551253, PMID:17328678 Sources: GOC:add